{
  "gene_symbol": "IFT52",
  "gene_name": "Intraflagellar transport protein 52 homolog",
  "term_id": "GO:0005929",
  "term_label": "cilium",
  "gene": "UniProtKB:Q9Y366"
}